transition metal ion transport [GO:0000041] (biological process) Relationships: is a type of metal ion transport [GO:0030001] Definition: The directed movement of transition metal ions into, out of or within a cell, or between cells, by means of some agent such as a transporter or pore. A transition metal is an element whose atom has an incomplete d-subshell of extranuclear electrons, or which gives rise to a cation or cations with an incomplete d-subshell. Transition metals often have more than one valency state. Biologically relevant transition metals include vanadium, manganese, iron, copper, cobalt, nickel, molybdenum and silver. Subtypes: cobalt ion transport [GO:0006824], GO:0006825, GO:0006826, manganese ion transport [GO:0006828], zinc ion transport [GO:0006829], silver ion transport [GO:0015673], GO:0015675, vanadium ion transport [GO:0015676], cadmium ion transport [GO:0015691], mercury ion transport [GO:0015694] Sources: ISBN:0198506732 Also known as: transition metal transport